{
  "gene_symbol": "TDRKH",
  "term_label": "spermatogenesis",
  "gene": "UniProtKB:Q9Y2W6",
  "gene_name": "Tudor and KH domain-containing protein",
  "term_id": "GO:0007283"
}